{
  "gene_name": "Protein shisa-like-1",
  "term_id": "UNKNOWN:0002",
  "gene_symbol": "SHISAL1",
  "gene": "UniProtKB:Q3SXP7",
  "term_label": "Unknown biological process"
}